{
  "term_id": "GO:0070382",
  "gene": "UniProtKB:Q9BSW7",
  "gene_name": "Synaptotagmin-17",
  "term_label": "exocytic vesicle",
  "gene_symbol": "SYT17"
}